structural constituent of eye lens [GO:0005212] (MF) Relationships: is_a structural molecule activity [GO:0005198] Definition: The action of a molecule that contributes to the structural integrity of the lens of an eye. Sources: GOC:mah